negative regulation of cell volume [GO:0045794] (biological process) Sources: GOC:go_curators Definition: Any process that decreases cell volume. Also known as: RVD, cell regulatory volume decrease Relationships: is a type of cell volume homeostasis [GO:0006884]